{
  "gene_symbol": "BTNL8",
  "term_id": "GO:0050852",
  "gene": "UniProtKB:Q6UX41",
  "term_label": "T cell receptor signaling pathway",
  "gene_name": "Butyrophilin-like protein 8"
}